{
  "gene": "UniProtKB:P10827",
  "term_label": "cell differentiation",
  "gene_symbol": "THRA",
  "gene_name": "Thyroid hormone receptor alpha",
  "term_id": "GO:0030154"
}